type 5A serotonin receptor binding [GO:0031830] (molecular function) Definition: Binding to a type 5A serotonin receptor. Relationships: is a type of G protein-coupled serotonin receptor binding [GO:0031821] Also known as: 5-hydroxytryptamine 5A receptor binding, type 5A serotonin receptor ligand Sources: GOC:mah, GOC:nln